protein folding [GO:0006457] (biological process) Sources: GOC:go_curators, GOC:rb Also known as: alpha-tubulin folding, beta-tubulin folding, chaperonin-mediated tubulin folding, chaperone activity, chaperonin ATPase activity, co-chaperone activity, co-chaperonin activity, glycoprotein-specific chaperone activity, non-chaperonin molecular chaperone ATPase activity, protein complex assembly, multichaperone pathway Subtypes: 'de novo' protein folding [GO:0006458], post-chaperonin tubulin folding pathway [GO:0007023], protein folding in endoplasmic reticulum [GO:0034975], GO:0042026, mitochondrial disulfide relay system [GO:0160203] Definition: The process of assisting in the covalent and noncovalent assembly of single chain polypeptides or multisubunit complexes into the correct tertiary structure. Relationships: is a type of cellular process [GO:0009987]; is part of protein maturation [GO:0051604] Regulation: RO_0002211 by GO:1903332; negatively regulated by GO:1903333; positively regulated by positive regulation of protein folding [GO:1903334]